disaccharide catabolic process [GO:0046352] (biological process) Definition: The chemical reactions and pathways resulting in the breakdown of disaccharides, sugars composed of two monosaccharide units. Sources: GOC:ai Also known as: disaccharide breakdown, disaccharide catabolism, disaccharide degradation Relationships: is a type of disaccharide metabolic process [GO:0005984]; is a type of oligosaccharide catabolic process [GO:0009313] Subtypes: maltose catabolic process [GO:0000025], sucrose catabolic process [GO:0005987], lactose catabolic process [GO:0005990], trehalose catabolic process [GO:0005993], GO:0005995, cellobiose catabolic process [GO:2000892]